oxidoreductase activity, acting on iron-sulfur proteins as donors, NAD or NADP as acceptor [GO:0016731] (molecular function) Sources: GOC:jl Definition: Catalysis of an oxidation-reduction (redox) reaction in which an iron-sulfur protein acts as a hydrogen or electron donor and reduces NAD or NADP. Relationships: is a type of GO:0016730 Subtypes: GO:0008937, rubredoxin-NAD(P)H reductase activity [GO:0015045], NADPH-iron-sulfur [2Fe-2S] protein oxidoreductase activity [GO:0160246]